{
  "term_label": "protein N-linked glycosylation",
  "gene_symbol": "MGAT5B",
  "gene_name": "Alpha-1,6-mannosylglycoprotein 6-beta-N-acetylglucosaminyltransferase B",
  "gene": "UniProtKB:Q3V5L5",
  "term_id": "GO:0006487"
}